regulation of mesonephros development [GO:0061217] (biological process) Subtypes: positive regulation of mesonephros development [GO:0061213], negative regulation of mesonephros development [GO:0061218], mesonephric renal vesicle induction [GO:0061294], GO:0072106, regulation of mesonephric glomerulus development [GO:2000087] Relationships: is a type of regulation of kidney development [GO:0090183]; regulates mesonephros development [GO:0001823] Definition: Any process that modulates the rate, frequency or extent of mesonephros development. Mesonephros development is the process whose specific outcome is the progression of the mesonephros over time, from its formation to the mature structure. The mesonephros is an endocrine and metabolic organ that filters the blood and excretes the end products of body metabolism in the form of urine. Sources: GOC:mtg_kidney_jan10